nuclear proteasome core complex, alpha-subunit complex [GO:0031604] (cellular component) Definition: The subunits forming the outer ring of the core complex of a proteasome located in the nucleus of a cell. Sources: GOC:mah Relationships: is a type of proteasome core complex, alpha-subunit complex [GO:0019773]; is a type of nuclear protein-containing complex [GO:0140513]; is part of nuclear proteasome core complex [GO:0031601]